{
  "gene_symbol": "REEP5",
  "gene_name": "Receptor expression-enhancing protein 5",
  "gene": "UniProtKB:Q00765",
  "term_label": "Unknown molecular function",
  "term_id": "UNKNOWN:0001"
}